{
  "gene_symbol": "MFHAS1",
  "gene": "UniProtKB:Q9Y4C4",
  "gene_name": "Malignant fibrous histiocytoma-amplified sequence 1",
  "term_id": "GO:0045087",
  "term_label": "innate immune response"
}